{
  "gene_symbol": "SLC26A5",
  "term_id": "GO:0007605",
  "gene_name": "Prestin",
  "gene": "UniProtKB:P58743",
  "term_label": "sensory perception of sound"
}